{
  "gene_name": "Paladin",
  "term_id": "GO:0005634",
  "gene_symbol": "PALD1",
  "term_label": "nucleus",
  "gene": "UniProtKB:Q9ULE6"
}